{
  "gene_name": "Solute carrier organic anion transporter family member 5A1",
  "gene_symbol": "SLCO5A1",
  "term_id": "GO:0016323",
  "term_label": "basolateral plasma membrane",
  "gene": "UniProtKB:Q9H2Y9"
}